{
  "gene_symbol": "ZFAND1",
  "term_label": "cytoplasm",
  "gene_name": "AN1-type zinc finger protein 1",
  "term_id": "GO:0005737",
  "gene": "UniProtKB:Q8TCF1"
}